{
  "gene_symbol": "EEF1DP3",
  "term_label": "Unknown cellular component",
  "gene_name": "Putative elongation factor 1-delta-like protein",
  "term_id": "UNKNOWN:0003",
  "gene": "UniProtKB:Q658K8"
}